somatic motor neuron differentiation [GO:0021523] (biological process) Relationships: is a type of GO:0021522 References: PMID:11262869 Sources: GOC:cls, GOC:dgh, GOC:dph, GOC:jid, GO_REF:0000021 Definition: The process in which neuroepithelial cells in the neural tube acquire specialized structural and/or functional features of somatic motor neurons. Somatic motor neurons innervate skeletal muscle targets and are responsible for transmission of motor impulses from the brain to the periphery. Differentiation includes the processes involved in commitment of a cell to a specific fate.